{
  "gene_symbol": "FAM223B",
  "term_label": "Unknown molecular function",
  "gene_name": "Protein FAM223B",
  "term_id": "UNKNOWN:0001",
  "gene": "UniProtKB:A6NKX1"
}